benzonitrile metabolic process [GO:0018876] (biological process) Also known as: benzonitrile metabolism Sources: UM-BBD_pathwayID:bzn Definition: The chemical reactions and pathways involving benzonitrile. Benzonitrile is used as a solvent and chemical intermediate in the pharmaceutical, dyestuffs and rubber industries. It is highly toxic and harmful in contact with skin. Relationships: is a type of benzene-containing compound metabolic process [GO:0042537]; is a type of GO:0050898